amphid sensory organ dendrite retrograde extension [GO:0003391] (biological process) Definition: The progression of an amphid sensory organ's neuronal dendrite over time by the attachment of a part of the cell to an anchor and the subsequent migration of the cell body away from the anchor point. Sources: GOC:ascb_2009, GOC:dph, GOC:tb Relationships: is a type of dendrite development by retrograde extension [GO:0003390]; is part of neuron development involved in amphid sensory organ development [GO:0003388]